{
  "term_id": "GO:0005768",
  "gene_name": "WASH complex subunit 4",
  "term_label": "endosome",
  "gene_symbol": "WASHC4",
  "gene": "UniProtKB:Q2M389"
}